{
  "gene_symbol": "PLCE1",
  "term_label": "G protein-coupled receptor signaling pathway",
  "term_id": "GO:0007186",
  "gene_name": "1-phosphatidylinositol 4,5-bisphosphate phosphodiesterase epsilon-1",
  "gene": "UniProtKB:Q9P212"
}